{
  "gene": "UniProtKB:Q13461",
  "gene_symbol": "FOXE3",
  "term_id": "GO:0000978",
  "gene_name": "Forkhead box protein E3",
  "term_label": "RNA polymerase II cis-regulatory region sequence-specific DNA binding"
}